{
  "gene_name": "Endothelial PAS domain-containing protein 1",
  "gene": "UniProtKB:Q99814",
  "gene_symbol": "EPAS1",
  "term_id": "GO:0071456",
  "term_label": "cellular response to hypoxia"
}